pentacyclic triterpenoid biosynthetic process [GO:0019745] (biological process) Relationships: is a type of GO:0016104; is a type of pentacyclic triterpenoid metabolic process [GO:0019742] Sources: ISBN:0198506732 Definition: The chemical reactions and pathways resulting in the formation of pentacyclic triterpenoid compounds, terpenoids with six isoprene units and 5 carbon rings. Subtypes: GO:1902383, GO:1902386 Also known as: pentacyclic triterpenoid anabolism, pentacyclic triterpenoid biosynthesis, pentacyclic triterpenoid formation, pentacyclic triterpenoid synthesis